{
  "gene": "UniProtKB:O95264",
  "gene_symbol": "HTR3B",
  "term_label": "synapse",
  "term_id": "GO:0045202",
  "gene_name": "5-hydroxytryptamine receptor 3B"
}